oxidoreductase activity, acting on a sulfur group of donors, cytochrome as acceptor [GO:0016669] (molecular function) Definition: Catalysis of an oxidation-reduction (redox) reaction in which a sulfur-containing group acts as a hydrogen or electron donor and reduces a cytochrome. Sources: GOC:jl Also known as: oxidoreductase activity, acting on sulphur group of donors, cytochrome as acceptor Relationships: is a type of oxidoreductase activity, acting on a sulfur group of donors [GO:0016667] Subtypes: GO:0050310, thiosulfate dehydrogenase activity [GO:0050338], sulfide dehydrogenase activity [GO:0070225]